{
  "term_id": "GO:0005789",
  "term_label": "endoplasmic reticulum membrane",
  "gene": "UniProtKB:P57057",
  "gene_name": "Glucose-6-phosphate exchanger SLC37A1",
  "gene_symbol": "SLC37A1"
}